venom-mediated edema [GO:0044398] (biological process) Definition: A process by which an organism causes swelling of soft tissues in another organism via the action of a venom. Edema is the result of excess water accumulation in tissues. References: PMID:20562011 Also known as: envenomation resulting in induction of edema in another organism, envenomation resulting in induction of edema in other organism, envenomation resulting in induction of oedema in other organism Relationships: is a type of venom-mediated perturbation of biological process [GO:0035738]